{
  "term_id": "GO:0009897",
  "gene_symbol": "CSF3R",
  "term_label": "external side of plasma membrane",
  "gene": "UniProtKB:Q99062",
  "gene_name": "Granulocyte colony-stimulating factor receptor"
}